positive regulation of endosome organization [GO:1904980] (biological process) Definition: Any process that activates or increases the frequency, rate or extent of endosome organization. References: PMID:22511594 Sources: GOC:PARL, GOC:TermGenie, GOC:pad, GO_REF:0000058 Also known as: positive regulation of endosome organisation, up regulation of endosome organisation, up regulation of endosome organization, up-regulation of endosome organisation, up-regulation of endosome organization, upregulation of endosome organisation, upregulation of endosome organization, activation of endosome organisation, activation of endosome organization, activation of endosome organization and biogenesis, positive regulation of endosome organization and biogenesis, up regulation of endosome organization and biogenesis, up-regulation of endosome organization and biogenesis, upregulation of endosome organization and biogenesis Relationships: is a type of positive regulation of organelle organization [GO:0010638]; is a type of GO:1904978; positively regulates endosome organization [GO:0007032] Subtypes: positive regulation of intralumenal vesicle formation [GO:1905367]